{
  "gene_symbol": "DLG4",
  "term_label": "neuron projection",
  "gene_name": "Disks large homolog 4",
  "gene": "UniProtKB:P78352",
  "term_id": "GO:0043005"
}